{
  "gene": "UniProtKB:O94782",
  "term_label": "cytosol",
  "gene_symbol": "USP1",
  "term_id": "GO:0005829",
  "gene_name": "Ubiquitin carboxyl-terminal hydrolase 1"
}